{
  "gene_symbol": "KEL",
  "term_label": "protein processing",
  "gene": "UniProtKB:P23276",
  "term_id": "GO:0016485",
  "gene_name": "Kell blood group glycoprotein"
}